{
  "gene_symbol": "UNC119",
  "gene_name": "Protein unc-119 homolog A",
  "term_label": "negative regulation of caveolin-mediated endocytosis",
  "term_id": "GO:2001287",
  "gene": "UniProtKB:Q13432"
}